{
  "gene_name": "Unconventional myosin-IXa",
  "gene_symbol": "MYO9A",
  "term_label": "actin filament binding",
  "term_id": "GO:0051015",
  "gene": "UniProtKB:B2RTY4"
}